{
  "gene": "UniProtKB:Q5TAH2",
  "gene_name": "Sodium_hydrogen exchanger 11",
  "gene_symbol": "SLC9C2",
  "term_label": "potassium ion transmembrane transport",
  "term_id": "GO:0071805"
}